muscle cell apoptotic process [GO:0010657] (biological process) Relationships: is a type of apoptotic process [GO:0006915] Subtypes: GO:0010658, GO:0034390 Definition: A form of programmed cell death induced by external or internal signals that trigger the activity of proteolytic caspases, whose actions dismantle a muscle cell and result in its death. A muscle cell is a mature contractile cell, commonly known as a myocyte, that forms one of three kinds of muscle. Regulation: negatively regulated by negative regulation of muscle cell apoptotic process [GO:0010656]; regulated by regulation of muscle cell apoptotic process [GO:0010660]; positively regulated by positive regulation of muscle cell apoptotic process [GO:0010661] Sources: CL:0000187, GOC:dph, GOC:mtg_apoptosis, GOC:tb Also known as: muscle cell apoptosis